{
  "gene_name": "Coactosin-like protein",
  "term_label": "regulation of actin filament polymerization",
  "term_id": "GO:0030833",
  "gene_symbol": "COTL1",
  "gene": "UniProtKB:Q14019"
}